{
  "gene_symbol": "SON",
  "gene": "UniProtKB:P18583",
  "term_id": "UNKNOWN:0003",
  "term_label": "Unknown cellular component",
  "gene_name": "Protein SON"
}